{
  "term_label": "rRNA (cytosine-N4-)-methyltransferase activity",
  "term_id": "GO:0071424",
  "gene_symbol": "METTL15",
  "gene": "UniProtKB:A6NJ78",
  "gene_name": "12S rRNA N4-methylcytidine (m4C) methyltransferase"
}